{
  "gene_symbol": "PIGS",
  "gene_name": "GPI transamidase component PIG-S",
  "term_label": "GPI-anchor transamidase complex",
  "term_id": "GO:0042765",
  "gene": "UniProtKB:Q96S52"
}